detection of mechanical stimulus involved in sensory perception of pain [GO:0050966] (BP) Sources: GOC:ai, GOC:dos Relationships: is a type of detection of mechanical stimulus involved in sensory perception [GO:0050974]; is a type of detection of stimulus involved in sensory perception of pain [GO:0062149] Also known as: perception of pain, detection of mechanical stimulus, perception of pain, sensory detection of mechanical stimulus, perception of pain, sensory transduction of mechanical stimulus, sensory detection of mechanical stimulus during perception of pain, sensory transduction of mechanical stimulus during perception of pain, mechanical nociception Definition: The series of events involved in the perception of pain in which a mechanical stimulus is received and converted into a molecular signal.